{
  "term_id": "GO:0042594",
  "gene_symbol": "ULK2",
  "gene_name": "Serine_threonine-protein kinase ULK2",
  "gene": "UniProtKB:Q8IYT8",
  "term_label": "response to starvation"
}